{
  "gene_name": "Speedy protein E1",
  "term_label": "protein kinase binding",
  "gene": "UniProtKB:Q8NFV5",
  "term_id": "GO:0019901",
  "gene_symbol": "SPDYE1"
}